{
  "gene_symbol": "HELB",
  "gene_name": "DNA helicase B",
  "term_label": "regulation of DNA double-strand break processing",
  "gene": "UniProtKB:Q8NG08",
  "term_id": "GO:1903775"
}